regulation of cellular response to growth factor stimulus [GO:0090287] (biological process) Relationships: is a type of GO:0048583; regulates cellular response to growth factor stimulus [GO:0071363] Subtypes: regulation of BMP signaling pathway [GO:0030510], regulation of vascular endothelial growth factor receptor signaling pathway [GO:0030947], regulation of fibroblast growth factor receptor signaling pathway [GO:0040036], regulation of neurotrophin TRK receptor signaling pathway [GO:0051386], negative regulation of cellular response to growth factor stimulus [GO:0090288], regulation of cellular response to vascular endothelial growth factor stimulus [GO:1902547], regulation of cellular response to transforming growth factor beta stimulus [GO:1903844], regulation of cell chemotaxis to fibroblast growth factor [GO:1904847], GO:2001112 Definition: Any process that modulates the rate, frequency, or extent of a change in state or activity of a cell (in terms of movement, secretion, enzyme production, gene expression, etc.) as a result of a growth factor stimulus. Sources: GOC:tb